{
  "term_id": "GO:0005615",
  "gene_name": "Retinoic acid receptor responder protein 2",
  "gene_symbol": "RARRES2",
  "gene": "UniProtKB:Q99969",
  "term_label": "extracellular space"
}